aromatic amino acid family biosynthetic process, prephenate pathway [GO:0009095] (biological process) Definition: The chemical reactions and pathways resulting in the formation of phenylalanine and tyrosine from other compounds, including chorismate, via the intermediate prephenate. Subtypes: L-tyrosine biosynthetic process [GO:0006571], L-phenylalanine biosynthetic process [GO:0009094] Also known as: aromatic amino acid family anabolism, prephenate pathway, aromatic amino acid family biosynthetic process via prephenate, aromatic amino acid family biosynthetic process via prephenate(2-), aromatic amino acid family formation, prephenate pathway, aromatic amino acid family synthesis, prephenate pathway Relationships: is a type of aromatic amino acid family biosynthetic process [GO:0009073] Sources: GOC:mah, ISBN:0471331309